{
  "gene_symbol": "CDC23",
  "gene": "UniProtKB:Q9UJX2",
  "term_label": "anaphase-promoting complex-dependent catabolic process",
  "gene_name": "Cell division cycle protein 23 homolog",
  "term_id": "GO:0031145"
}